imidazolonepropionase activity [GO:0050480] (molecular function) Definition: Catalysis of the reaction: (S)-3-(4-oxo-4,5-dihydro-1H-imidazol-5-yl)propanoic acid + H2O = N-formimidoyl-L-glutamate + H+. Relationships: is a type of hydrolase activity, acting on carbon-nitrogen (but not peptide) bonds, in cyclic amides [GO:0016812] Sources: EC:3.5.2.7, RHEA:23660 Also known as: 3-(5-oxo-4,5-dihydro-3H-imidazol-4-yl)propanoate amidohydrolase activity, 4(5)-imidazolone-5(4)-propionic acid hydrolase activity, imidazolone propionic acid hydrolase activity, imidazolone-5-propionate hydrolase activity